{
  "gene_name": "Leucine-rich repeat-containing protein 51",
  "gene_symbol": "LRRC51",
  "gene": "UniProtKB:Q96E66",
  "term_id": "UNKNOWN:0001",
  "term_label": "Unknown molecular function"
}